{
  "gene": "UniProtKB:P57053",
  "gene_symbol": "H2BC12L",
  "term_id": "GO:0005615",
  "gene_name": "Histone H2B type F-S",
  "term_label": "extracellular space"
}